{
  "gene_name": "Arf-GAP with GTPase, ANK repeat and PH domain-containing protein 5",
  "gene": "UniProtKB:A6NIR3",
  "term_id": "UNKNOWN:0003",
  "gene_symbol": "AGAP5",
  "term_label": "Unknown cellular component"
}